{
  "gene_name": "tRNA (cytosine(72)-C(5))-methyltransferase NSUN6",
  "term_label": "Unknown molecular function",
  "term_id": "UNKNOWN:0001",
  "gene": "UniProtKB:Q8TEA1",
  "gene_symbol": "NSUN6"
}